{
  "gene_symbol": "CD1D",
  "term_id": "GO:0048006",
  "term_label": "antigen processing and presentation, endogenous lipid antigen via MHC class Ib",
  "gene": "UniProtKB:P15813",
  "gene_name": "Antigen-presenting glycoprotein CD1d"
}